{
  "gene_symbol": "ZNF497",
  "gene": "UniProtKB:Q6ZNH5",
  "term_id": "GO:0000978",
  "term_label": "RNA polymerase II cis-regulatory region sequence-specific DNA binding",
  "gene_name": "Zinc finger protein 497"
}